{
  "gene_symbol": "RBMX2",
  "term_label": "Unknown molecular function",
  "gene_name": "RNA-binding motif protein, X-linked 2",
  "gene": "UniProtKB:Q9Y388",
  "term_id": "UNKNOWN:0001"
}